{
  "gene": "UniProtKB:P53367",
  "term_label": "intracellular protein transport",
  "gene_symbol": "ARFIP1",
  "term_id": "GO:0006886",
  "gene_name": "Arfaptin-1"
}